{
  "gene_name": "KH domain-containing, RNA-binding, signal transduction-associated protein 3",
  "term_id": "GO:0003729",
  "gene_symbol": "KHDRBS3",
  "term_label": "mRNA binding",
  "gene": "UniProtKB:O75525"
}